P2Y9 nucleotide receptor binding [GO:0031818] (molecular function) Sources: GOC:mah, GOC:nln Also known as: P2Y9 nucleotide receptor ligand Relationships: is a type of G protein-coupled nucleotide receptor binding [GO:0031811] Definition: Binding to a P2Y9 nucleotide receptor.